dCMP catabolic process [GO:0006249] (biological process) Also known as: dCMP breakdown, dCMP catabolism, dCMP degradation Sources: ISBN:0198506732 Definition: The chemical reactions and pathways resulting in the breakdown of dCMP, deoxycytidine monophosphate. Relationships: is a type of pyrimidine deoxyribonucleoside monophosphate catabolic process [GO:0009178]; is a type of GO:0009223; is a type of GO:0046063